5S class rRNA transcription by RNA polymerase III [GO:0042791] (biological process) Also known as: 5S rRNA transcription, 5S class rRNA transcription from RNA polymerase III type 1 promoter Relationships: is a type of transcription by RNA polymerase III [GO:0006383]; is a type of rRNA transcription [GO:0009303] Definition: The synthesis of 5S ribosomal RNA (rRNA), or an equivalent rRNA, from a DNA template by RNA polymerase III (Pol III), originating at a type 1 RNA polymerase III promoter. References: PMID:12381659 Sources: GOC:jl, GOC:txnOH, ISBN:0321000382